{
  "gene_symbol": "ATP6V1C2",
  "term_label": "Unknown biological process",
  "gene": "UniProtKB:Q8NEY4",
  "term_id": "UNKNOWN:0002",
  "gene_name": "V-type proton ATPase subunit C 2"
}